{
  "term_id": "GO:0048813",
  "term_label": "dendrite morphogenesis",
  "gene_symbol": "TMEM106B",
  "gene": "UniProtKB:Q9NUM4",
  "gene_name": "Transmembrane protein 106B"
}